{
  "term_id": "GO:0031054",
  "gene_symbol": "AGO4",
  "term_label": "pre-miRNA processing",
  "gene_name": "Protein argonaute-4",
  "gene": "UniProtKB:Q9HCK5"
}